{
  "gene_name": "Dystrobrevin alpha",
  "gene": "UniProtKB:Q9Y4J8",
  "gene_symbol": "DTNA",
  "term_label": "synaptic signaling",
  "term_id": "GO:0099536"
}